{
  "gene_symbol": "SLC4A9",
  "gene": "UniProtKB:Q96Q91",
  "gene_name": "Anion exchange protein 4",
  "term_label": "transmembrane transport",
  "term_id": "GO:0055085"
}